{
  "gene_symbol": "CDK8",
  "gene_name": "Cyclin-dependent kinase 8",
  "term_id": "GO:1990508",
  "gene": "UniProtKB:P49336",
  "term_label": "CKM complex"
}